structural constituent of egg chorion [GO:0005213] (molecular function) Relationships: is a type of structural molecule activity [GO:0005198]; occurs in egg chorion [GO:0042600] Definition: The action of a molecule that contributes to the structural integrity of an egg chorion. An example of this is found in Drosophila melanogaster. Sources: GOC:mah, GOC:sensu Also known as: structural constituent of chorion, structural protein of chorion